{
  "term_label": "glucose homeostasis",
  "gene_name": "DNA-binding protein RFX6",
  "term_id": "GO:0042593",
  "gene": "UniProtKB:Q8HWS3",
  "gene_symbol": "RFX6"
}